{
  "term_label": "Unknown cellular component",
  "gene_name": "Ankyrin repeat and SOCS box protein 7",
  "gene": "UniProtKB:Q9H672",
  "term_id": "UNKNOWN:0003",
  "gene_symbol": "ASB7"
}